{
  "term_label": "late endosome",
  "term_id": "GO:0005770",
  "gene_name": "Cation-dependent mannose-6-phosphate receptor",
  "gene": "UniProtKB:P20645",
  "gene_symbol": "M6PR"
}